detection of hormone stimulus [GO:0009720] (biological process) Sources: GOC:sm Also known as: perception of hormone stimulus Definition: The series of events in which a hormone stimulus is received by a cell and converted into a molecular signal. Subtypes: detection of auxin stimulus [GO:0009721], detection of cytokinin stimulus [GO:0009722], detection of abscisic acid stimulus [GO:0009724], GO:0009727, detection of gibberellic acid stimulus [GO:0009728], detection of brassinosteroid stimulus [GO:0009729], detection of steroid hormone stimulus [GO:0051467] Relationships: is a type of GO:0009593; is a type of response to hormone [GO:0009725]